dendritic cell antigen processing and presentation [GO:0002468] (biological process) References: PMID:15771591 Sources: GOC:add, ISBN:0781735149 Relationships: is a type of antigen processing and presentation [GO:0019882] Regulation: regulated by regulation of dendritic cell antigen processing and presentation [GO:0002604]; negatively regulated by negative regulation of dendritic cell antigen processing and presentation [GO:0002605]; positively regulated by positive regulation of dendritic cell antigen processing and presentation [GO:0002606] Definition: The process in which a dendritic cell expresses antigen (peptide or lipid) on its cell surface in association with an MHC protein complex. Subtypes: GO:0002469, plasmacytoid dendritic cell antigen processing and presentation [GO:0002470]